{
  "gene_name": "Intraflagellar transport protein 46 homolog",
  "gene": "UniProtKB:Q9NQC8",
  "gene_symbol": "IFT46",
  "term_id": "GO:0030992",
  "term_label": "intraciliary transport particle B"
}